{
  "gene_symbol": "ASCC2",
  "gene_name": "Activating signal cointegrator 1 complex subunit 2",
  "term_id": "GO:0043130",
  "term_label": "ubiquitin binding",
  "gene": "UniProtKB:Q9H1I8"
}